{
  "gene_symbol": "FERMT2",
  "gene_name": "Fermitin family homolog 2",
  "term_label": "integrin binding",
  "gene": "UniProtKB:Q96AC1",
  "term_id": "GO:0005178"
}